positive regulation of endocardial cushion cell differentiation [GO:0120075] (BP) Sources: GOC:BHF, GOC:BHF_miRNA, GOC:rph Relationships: is a type of regulation of endocardial cushion cell differentiation [GO:0120074]; is a type of GO:1905209; positively regulates GO:0061443 Definition: Any process that activates or increases the frequency, rate or extent of endocardial cushion cell differentiation.